{
  "term_id": "GO:0016604",
  "term_label": "nuclear body",
  "gene": "UniProtKB:Q9H9A7",
  "gene_name": "RecQ-mediated genome instability protein 1",
  "gene_symbol": "RMI1"
}